{
  "term_id": "GO:0004714",
  "term_label": "transmembrane receptor protein tyrosine kinase activity",
  "gene_name": "Proto-oncogene tyrosine-protein kinase ROS",
  "gene": "UniProtKB:P08922",
  "gene_symbol": "ROS1"
}